{
  "gene_symbol": "GDAP2",
  "gene": "UniProtKB:Q9NXN4",
  "gene_name": "Ganglioside-induced differentiation-associated protein 2",
  "term_id": "UNKNOWN:0001",
  "term_label": "Unknown molecular function"
}